{
  "term_id": "GO:0006891",
  "gene_symbol": "RAB6A",
  "gene_name": "Ras-related protein Rab-6A",
  "term_label": "intra-Golgi vesicle-mediated transport",
  "gene": "UniProtKB:P20340"
}